interleukin-34-mediated signaling pathway [GO:0061514] (biological process) Definition: The series of molecular signals initiated by interleukin-34 binding to its receptor on the surface of a target cell, and ending with the regulation of a downstream cellular process, e.g. transcription. Relationships: is a type of GO:0019221 References: PMID:18467591 Sources: GOC:dph